{
  "gene_symbol": "MT-ATP8",
  "gene": "UniProtKB:P03928",
  "term_id": "GO:0045259",
  "term_label": "proton-transporting ATP synthase complex",
  "gene_name": "ATP synthase protein 8"
}